{
  "gene_name": "CTD small phosphatase-like protein",
  "term_id": "GO:0008420",
  "gene": "UniProtKB:O15194",
  "term_label": "RNA polymerase II CTD heptapeptide repeat phosphatase activity",
  "gene_symbol": "CTDSPL"
}